tRNA-derived regulatory ncRNA processing [GO:0140891] (biological process) References: PMID:29120263 Definition: A process leading to the generation of a functional small regulatory non-coding RNA derived from a tRNA. Relationships: is a type of GO:0070918 Also known as: tRNA-derived small RNA processing